mastication [GO:0071626] (biological process) Sources: GOC:gvg Definition: The process of biting and mashing food with the teeth prior to swallowing. Also known as: chewing Relationships: is a type of digestive system process [GO:0022600]